macropinocytic cup cytoskeleton [GO:0070687] (cellular component) Sources: GOC:mah Also known as: crown cytoskeleton Relationships: is a type of cellular anatomical structure [GO:0110165]; is part of cortical actin cytoskeleton [GO:0030864]; is part of GO:0070685 Definition: The part of the cortical actin cytoskeleton that forms part of a macropinocytic cup.